{
  "gene_symbol": "ACAN",
  "term_id": "GO:0072534",
  "term_label": "perineuronal net",
  "gene_name": "Aggrecan core protein",
  "gene": "UniProtKB:P16112"
}